{
  "gene": "UniProtKB:Q9Y5L4",
  "gene_symbol": "TIMM13",
  "term_label": "mitochondrial intermembrane space chaperone complex",
  "gene_name": "Mitochondrial import inner membrane translocase subunit Tim13",
  "term_id": "GO:0042719"
}